interleukin-24 receptor activity [GO:0045506] (molecular function) Definition: Combining with interleukin-24 and transmitting the signal from one side of the membrane to the other to initiate a change in cell activity. Sources: GOC:jl, GOC:signaling Also known as: IL-24 receptor activity, IL-24R Relationships: is a type of cytokine receptor activity [GO:0004896]; has part interleukin-24 binding [GO:0045510]